regulation of protein import into nucleus [GO:0042306] (biological process) Relationships: is a type of regulation of intracellular protein transport [GO:0033157]; is a type of regulation of nucleocytoplasmic transport [GO:0046822]; is a type of regulation of protein localization to nucleus [GO:1900180]; regulates GO:0006606 Also known as: regulation of protein import into cell nucleus, regulation of protein transport from cytoplasm to nucleus, regulation of protein-nucleus import Sources: GOC:jl Definition: Any process that modulates the frequency, rate or extent of movement of proteins from the cytoplasm to the nucleus. Subtypes: positive regulation of protein import into nucleus [GO:0042307], GO:0042308